{
  "term_id": "GO:0005737",
  "gene_symbol": "RNF34",
  "gene_name": "E3 ubiquitin-protein ligase RNF34",
  "term_label": "cytoplasm",
  "gene": "UniProtKB:Q969K3"
}